male courtship behavior, veined wing generated song production [GO:0045433] (biological process) Relationships: is a type of male courtship behavior [GO:0008049]; BFO_0000050 male courtship behavior, veined wing vibration [GO:0016545] References: PMID:11092827 Sources: GOC:mtg_sensu Definition: The process during wing vibration where the male insect produces a species-specific acoustic signal called a love song. Also known as: male courtship behavior, song production, male courtship behaviour, song production, male courtship behaviour, veined wing generated song production